Lewy body [GO:0097413] (cellular component) Sources: NIF_Subcellular:sao4933778419 Relationships: is a type of GO:0016234 Definition: Cytoplasmic, spherical inclusion commonly found in damaged neurons, and composed of abnormally phosphorylated, neurofilament proteins aggregated with ubiquitin and alpha-synuclein. Also known as: cytoplasmic inclusion Subtypes: classical Lewy body [GO:0097414], cortical Lewy body [GO:0097415]